lung cell differentiation [GO:0060479] (biological process) Definition: The process in which relatively unspecialized cells, e.g. embryonic or regenerative cells, acquire specialized structural and/or functional features of a mature cell found in the lung. Differentiation includes the processes involved in commitment of a cell to a specific fate. Relationships: is a type of cell differentiation [GO:0030154]; BFO_0000050 lung development [GO:0030324] Subtypes: lung epithelial cell differentiation [GO:0060487], lung basal cell differentiation [GO:0060508] Sources: GOC:dph, GOC:mtg_lung Also known as: pulmonary cell differentiation